{
  "term_label": "RNA polymerase II cis-regulatory region sequence-specific DNA binding",
  "term_id": "GO:0000978",
  "gene_symbol": "ZNF12",
  "gene": "UniProtKB:P17014",
  "gene_name": "Zinc finger protein 12"
}